{
  "gene": "UniProtKB:Q92859",
  "gene_symbol": "NEO1",
  "term_label": "cell surface",
  "term_id": "GO:0009986",
  "gene_name": "Neogenin"
}